{
  "gene_name": "E3 ubiquitin ligase TRIM40",
  "term_id": "GO:0061630",
  "gene_symbol": "TRIM40",
  "term_label": "ubiquitin protein ligase activity",
  "gene": "UniProtKB:Q6P9F5"
}